{
  "gene": "UniProtKB:Q6Y7W6",
  "gene_symbol": "GIGYF2",
  "term_id": "GO:0045947",
  "gene_name": "GRB10-interacting GYF protein 2",
  "term_label": "negative regulation of translational initiation"
}